{
  "term_id": "GO:0032446",
  "gene": "UniProtKB:O95352",
  "gene_name": "Ubiquitin-like modifier-activating enzyme ATG7",
  "term_label": "protein modification by small protein conjugation",
  "gene_symbol": "ATG7"
}